{
  "term_label": "cytosol",
  "gene_name": "A-kinase anchor protein 17A",
  "gene_symbol": "AKAP17A",
  "term_id": "GO:0005829",
  "gene": "UniProtKB:Q02040"
}